sperm plasma membrane [GO:0097524] (cellular component) Sources: GOC:cjm Relationships: is a type of plasma membrane [GO:0005886] Definition: A plasma membrane that is part of a sperm cell.